{
  "gene_symbol": "PITPNM2",
  "gene": "UniProtKB:Q9BZ72",
  "term_id": "UNKNOWN:0002",
  "term_label": "Unknown biological process",
  "gene_name": "Membrane-associated phosphatidylinositol transfer protein 2"
}